{
  "term_id": "GO:0006888",
  "term_label": "endoplasmic reticulum to Golgi vesicle-mediated transport",
  "gene_symbol": "YIPF5",
  "gene_name": "Protein YIPF5",
  "gene": "UniProtKB:Q969M3"
}